{
  "gene_symbol": "GALNTL5",
  "term_label": "Golgi apparatus",
  "term_id": "GO:0005794",
  "gene_name": "Inactive polypeptide N-acetylgalactosaminyltransferase-like protein 5",
  "gene": "UniProtKB:Q7Z4T8"
}